{
  "term_id": "UNKNOWN:0002",
  "gene_name": "Clusterin-like protein 1",
  "gene": "UniProtKB:Q15846",
  "gene_symbol": "CLUL1",
  "term_label": "Unknown biological process"
}